{
  "term_id": "GO:0022841",
  "gene": "UniProtKB:Q9HB15",
  "gene_name": "Potassium channel subfamily K member 12",
  "gene_symbol": "KCNK12",
  "term_label": "potassium ion leak channel activity"
}